{
  "gene_name": "G1_S-specific cyclin-D1",
  "gene_symbol": "CCND1",
  "term_label": "microtubule organizing center",
  "gene": "UniProtKB:P24385",
  "term_id": "GO:0005815"
}